nicotinic acid riboside biosynthetic process [GO:0071592] (biological process) Relationships: is a type of pyridine nucleoside biosynthetic process [GO:0071589] Definition: The chemical reactions and pathways resulting in the formation of nicotinic acid riboside, the product of the formation of a glycosidic bond between ribose and nicotinic acid. References: PMID:19846558 Sources: GOC:mah Also known as: D-ribosylnicotinic acid biosynthetic process, nicotinic acid riboside anabolism, nicotinic acid riboside biosynthesis, nicotinic acid riboside formation, nicotinic acid riboside synthesis